positive regulation of cortisol biosynthetic process [GO:2000066] (biological process) Sources: GOC:obol, GOC:yaf Also known as: positive regulation of cortisol biosynthesis, positive regulation of cortisol formation, positive regulation of cortisol synthesis, positive regulation of cortisol anabolism Definition: Any process that activates or increases the frequency, rate or extent of cortisol biosynthetic process. Relationships: is a type of positive regulation of glucocorticoid biosynthetic process [GO:0031948]; is a type of positive regulation of alcohol biosynthetic process [GO:1902932]; is a type of GO:2000064; positively regulates cortisol biosynthetic process [GO:0034651]